{
  "gene": "UniProtKB:A6NGN9",
  "gene_symbol": "IGLON5",
  "term_label": "plasma membrane",
  "term_id": "GO:0005886",
  "gene_name": "IgLON family member 5"
}